{
  "gene_symbol": "UNC5A",
  "term_label": "netrin receptor activity",
  "term_id": "GO:0005042",
  "gene_name": "Netrin receptor UNC5A",
  "gene": "UniProtKB:Q6ZN44"
}